{
  "gene": "UniProtKB:Q9NQ66",
  "term_label": "calmodulin binding",
  "gene_name": "1-phosphatidylinositol 4,5-bisphosphate phosphodiesterase beta-1",
  "term_id": "GO:0005516",
  "gene_symbol": "PLCB1"
}